mannan endo-1,4-beta-mannosidase activity [GO:0016985] (molecular function) Also known as: beta-mannanase activity, endo-1,4-mannanase activity, endo-beta-mannanase activity, 1,4-beta-D-mannan mannanohydrolase activity, beta-1,4-mannan 4-mannanohydrolase activity, beta-D-mannanase activity, beta-mannanase B, endo-1,4-beta-mannanase activity, endo-beta-1,4-mannase activity Sources: EC:3.2.1.78 Definition: Catalysis of the random hydrolysis of (1->4)-beta-D-mannosidic linkages in mannans, galactomannans, glucomannans, and galactoglucomannans. Relationships: is a type of beta-mannosidase activity [GO:0004567]